site of polarized growth [GO:0030427] (cellular component) Relationships: is a type of cellular anatomical structure [GO:0110165] Subtypes: incipient cellular bud site [GO:0000131], hyphal tip [GO:0001411], cellular bud tip [GO:0005934], cellular bud neck [GO:0005935], growth cone [GO:0030426], growing cell tip [GO:0035838], mating projection tip [GO:0043332] Definition: Any part of a cell where non-isotropic growth takes place. Sources: GOC:mah